vesicle fusion with endoplasmic reticulum [GO:0048279] (biological process) Definition: The joining of the lipid bilayer membrane around a vesicle to the lipid bilayer membrane around the endoplasmic reticulum. Sources: GOC:jid Also known as: vesicle fusion with ER Subtypes: endoplasmic reticulum-Golgi intermediate compartment (ERGIC) derived vesicle fusion with endoplasmic reticulum membrane [GO:1990669] Relationships: is a type of GO:0006906; is a type of endoplasmic reticulum organization [GO:0007029]